{
  "gene_name": "DNA replication factor Cdt1",
  "term_label": "mitotic cell cycle",
  "term_id": "GO:0000278",
  "gene": "UniProtKB:Q9H211",
  "gene_symbol": "CDT1"
}